oxidoreductase activity, acting on the CH-NH group of donors, NAD or NADP as acceptor [GO:0016646] (molecular function) Definition: Catalysis of an oxidation-reduction (redox) reaction in which a CH-NH group acts as a hydrogen or electron donor and reduces NAD or NADP. Relationships: is a type of oxidoreductase activity, acting on the CH-NH group of donors [GO:0016645] Sources: GOC:jl Subtypes: dihydrofolate reductase activity [GO:0004146], GO:0004155, GO:0004487, GO:0004488, methylenetetrahydrofolate reductase [NAD(P)H] activity [GO:0004489], GO:0004735, saccharopine dehydrogenase activity [GO:0004753], FMN reductase [NAD(P)H] activity [GO:0008752], GO:0016155, folate reductase activity [GO:0033560], GO:0033739, flavin reductase (NADH) activity [GO:0036382], GO:0044684, pteridine reductase activity [GO:0047040], delta1-piperideine-2-carboxylate reductase activity [GO:0047125], N5-(carboxyethyl)ornithine synthase activity [GO:0047126], thiomorpholine-carboxylate dehydrogenase activity [GO:0047127], 1,2-dehydroreticulinium reductase (NADPH) activity [GO:0047128], GO:0047129, GO:0047636, GO:0047697, GO:0047827, GO:0047829, D-octopine dehydrogenase activity [GO:0047830], ephedrine dehydrogenase activity [GO:0047877], GO:0050241, strombine dehydrogenase activity [GO:0050305], tauropine dehydrogenase activity [GO:0050325], berberine reductase activity [GO:0050623], GO:0050624, riboflavin reductase [NAD(P)H] activity [GO:0052875], dehydropipecolic acid reductase [GO:0062046], dihydromonapterin reductase activity [GO:0071172], carboxynorspermidine dehydrogenase activity [GO:0102143], 8-hydroxy-5-deazaflavin:NADPH oxidoreductase activity [GO:0102261]